{
  "term_id": "UNKNOWN:0003",
  "gene": "UniProtKB:Q9GZT3",
  "term_label": "Unknown cellular component",
  "gene_name": "SRA stem-loop-interacting RNA-binding protein, mitochondrial",
  "gene_symbol": "SLIRP"
}